{
  "term_label": "Unknown cellular component",
  "term_id": "UNKNOWN:0003",
  "gene_symbol": "CAPN7",
  "gene": "UniProtKB:Q9Y6W3",
  "gene_name": "Calpain-7"
}